{
  "term_label": "negative regulation of cell population proliferation",
  "gene_symbol": "NUPR2",
  "gene": "UniProtKB:A6NF83",
  "gene_name": "Nuclear protein 2",
  "term_id": "GO:0008285"
}